dimethylglycine N-methyltransferase activity [GO:0052729] (molecular function) Relationships: is a type of N-methyltransferase activity [GO:0008170]; is a type of S-adenosylmethionine-dependent methyltransferase activity [GO:0008757] Definition: Catalysis of the reaction: S-adenosyl-L-methionine + N,N-dimethylglycine = S-adenosyl-L-homocysteine + betaine. Sources: RHEA:10072 Also known as: ApDMT, S-adenosyl-L-methionine:N,N-dimethylglycine N-methyltransferase activity